fetal process involved in parturition [GO:0060138] (biological process) Sources: GOC:dph Definition: A reproductive process occurring in the embryo that results in birth. Relationships: is a type of multicellular organismal reproductive process [GO:0048609]; is part of parturition [GO:0007567]; is part of embryo development ending in birth or egg hatching [GO:0009792]